{
  "term_label": "DNA helicase activity",
  "term_id": "GO:0003678",
  "gene": "UniProtKB:Q9H2U1",
  "gene_symbol": "DHX36",
  "gene_name": "ATP-dependent DNA_RNA helicase DHX36"
}